{
  "term_id": "UNKNOWN:0001",
  "gene": "UniProtKB:Q13522",
  "gene_symbol": "PPP1R1A",
  "term_label": "Unknown molecular function",
  "gene_name": "Protein phosphatase 1 regulatory subunit 1A"
}